{
  "term_label": "RNA binding",
  "term_id": "GO:0003723",
  "gene_name": "FAST kinase domain-containing protein 3, mitochondrial",
  "gene": "UniProtKB:Q14CZ7",
  "gene_symbol": "FASTKD3"
}